cell proliferation involved in imaginal disc-derived wing morphogenesis [GO:0090255] (BP) Sources: GOC:ascb_2009, GOC:dph, GOC:tb Definition: The multiplication or reproduction of cells, resulting in the expansion of a cell population that contributes to imaginal disc-derived wing morphogenesis. Regulation: regulated by GO:0090256 Relationships: is a type of cell population proliferation [GO:0008283]; is part of GO:0007476